purine deoxyribonucleoside metabolic process [GO:0046122] (biological process) Definition: The chemical reactions and pathways involving any one of a family of organic molecules consisting of a purine base covalently bonded to a sugar deoxyribose (a deoxyribonucleoside). Sources: GOC:ai Also known as: purine deoxyribonucleoside metabolism Relationships: is a type of deoxyribonucleoside metabolic process [GO:0009120]; is_a purine nucleoside metabolic process [GO:0042278] Subtypes: purine deoxyribonucleoside interconversion [GO:0019688], deoxyadenosine metabolic process [GO:0046090], GO:0046094, purine deoxyribonucleoside biosynthetic process [GO:0046123], purine deoxyribonucleoside catabolic process [GO:0046124]